{
  "term_label": "XPC complex",
  "gene_name": "DNA repair protein complementing XP-C cells",
  "term_id": "GO:0071942",
  "gene_symbol": "XPC",
  "gene": "UniProtKB:Q01831"
}